{
  "term_label": "plasma membrane",
  "gene_symbol": "ARL4D",
  "gene_name": "ADP-ribosylation factor-like protein 4D",
  "gene": "UniProtKB:P49703",
  "term_id": "GO:0005886"
}